alpha4-beta1 integrin-thrombospondin-1 complex [GO:0071069] (cellular component) Definition: A protein complex that consists of an alpha4-beta1 integrin complex bound to thrombospondin-1. Also known as: ITGA4-ITGB1-THBS1 complex Relationships: is a type of plasma membrane protein complex [GO:0098797] References: PMID:11980922